{
  "term_label": "olfactory receptor binding",
  "gene": "UniProtKB:P59025",
  "gene_name": "Receptor-transporting protein 1",
  "term_id": "GO:0031849",
  "gene_symbol": "RTP1"
}